positive regulation of sodium:proton antiporter activity [GO:0032417] (biological process) Relationships: is a type of GO:2000651; positively regulates sodium:proton antiporter activity [GO:0015385] Sources: GOC:mah Also known as: positive regulation of sodium:hydrogen antiporter activity, up regulation of sodium:hydrogen antiporter activity, up-regulation of sodium:hydrogen antiporter activity, upregulation of sodium:hydrogen antiporter activity, activation of sodium:hydrogen antiporter activity, stimulation of sodium:hydrogen antiporter activity Definition: Any process that activates or increases the activity of a sodium:hydrogen antiporter, which catalyzes the reaction: Na+(out) + H+(in) = Na+(in) + H+(out).